{
  "term_id": "GO:0019886",
  "gene_name": "HLA class II histocompatibility antigen, DR beta 5 chain",
  "gene_symbol": "HLA-DRB5",
  "term_label": "antigen processing and presentation of exogenous peptide antigen via MHC class II",
  "gene": "UniProtKB:Q30154"
}